{
  "term_label": "regulation of cell migration",
  "gene_symbol": "PLXND1",
  "term_id": "GO:0030334",
  "gene": "UniProtKB:Q9Y4D7",
  "gene_name": "Plexin-D1"
}